{
  "gene_symbol": "ZNF621",
  "gene": "UniProtKB:Q6ZSS3",
  "gene_name": "Zinc finger protein 621",
  "term_id": "GO:0006357",
  "term_label": "regulation of transcription by RNA polymerase II"
}